regulation of action potential [GO:0098900] (biological process) Definition: Any process that modulates the frequency, rate or extent of action potential creation, propagation or termination. This typically occurs via modulation of the activity or expression of voltage-gated ion channels. Note: The ion channels through which current flows during an action potential should be annotated to the process 'action potential'. Gene products involved in modulating the characteristics of an action potential via changing the expression levels or the activity of these channels (e.g. modulating their kinetics or voltage sensitivity) should be annotated to this regulation term. Sources: GOC:dos, GOC:dph, GOC:go_curators, GOC:tb, ISBN:978-0-07-139011-8 Subtypes: regulation of skeletal muscle contraction via regulation of action potential [GO:0014861], negative regulation of action potential [GO:0045759], positive regulation of action potential [GO:0045760], regulation of cardiac muscle cell action potential [GO:0098901], regulation of membrane repolarization during action potential [GO:0098903], regulation of neuronal action potential [GO:0098908], regulation of action potential firing rate [GO:0099605], GO:0099608, regulation of action potential firing threshold [GO:0099611] Relationships: is a type of regulation of membrane potential [GO:0042391]; is a type of GO:0050789; regulates GO:0001508